nitrobenzene nitroreductase (NADPH) activity [GO:0018546] (molecular function) Definition: Catalysis of the reaction: H2O + N-phenylhydroxylamine + 2 NADP+ = 2 H+ + 2 NADPH + nitrobenzene. References: PMID:16517619 Sources: RHEA:52884 Relationships: is a type of oxidoreductase activity, acting on other nitrogenous compounds as donors, with NAD or NADP as acceptor [GO:0046857]